{
  "gene_name": "Inorganic pyrophosphatase",
  "term_id": "GO:0006796",
  "term_label": "phosphate-containing compound metabolic process",
  "gene": "UniProtKB:Q15181",
  "gene_symbol": "PPA1"
}